{
  "gene_symbol": "BDH1",
  "term_id": "GO:0003858",
  "gene_name": "D-beta-hydroxybutyrate dehydrogenase, mitochondrial",
  "term_label": "3-hydroxybutyrate dehydrogenase activity",
  "gene": "UniProtKB:Q02338"
}